{
  "term_id": "UNKNOWN:0002",
  "term_label": "Unknown biological process",
  "gene": "UniProtKB:Q4JDL3",
  "gene_name": "Tyrosine-protein phosphatase non-receptor type 20",
  "gene_symbol": "PTPN20"
}